{
  "gene_symbol": "BRF2",
  "gene_name": "Transcription factor IIIB 50 kDa subunit",
  "gene": "UniProtKB:Q9HAW0",
  "term_id": "GO:0016251",
  "term_label": "RNA polymerase II general transcription initiation factor activity"
}